{
  "gene": "UniProtKB:Q05996",
  "gene_name": "Zona pellucida sperm-binding protein 2",
  "gene_symbol": "ZP2",
  "term_label": "prevention of polyspermy",
  "term_id": "GO:0060468"
}